response to far red light [GO:0010218] (BP) Relationships: is a type of response to red or far red light [GO:0009639] Subtypes: response to continuous far red light stimulus by the high-irradiance response system [GO:0010201], cellular response to far red light [GO:0071490] Sources: GOC:mtg_far_red, GOC:tb Also known as: response to far red light stimulus Definition: Any process that results in a change in state or activity of a cell or an organism (in terms of movement, secretion, enzyme production, gene expression, etc.) as a result of far red light stimulus. Far red light is electromagnetic radiation of wavelength 700-800nm. An example of this response is seen at the beginning of many plant species developmental stages. These include germination, and the point when cotyledon expansion is triggered. In certain species these processes take place in response to absorption of red light by the pigment molecule phytochrome, but the signal can be reversed by exposure to far red light. During the initial phase the phytochrome molecule is only present in the red light absorbing form, but on absorption of red light it changes to a far red light absorbing form, triggering progress through development. An immediate short period of exposure to far red light entirely returns the pigment to its initial state and prevents triggering of the developmental process. A thirty minute break between red and subsequent far red light exposure renders the red light effect irreversible, and development then occurs regardless of whether far red light exposure subsequently occurs.